{
  "gene_name": "Rhodopsin kinase GRK1",
  "term_id": "GO:0050254",
  "term_label": "rhodopsin kinase activity",
  "gene": "UniProtKB:Q15835",
  "gene_symbol": "GRK1"
}